larval chitin-based cuticle development [GO:0008363] (biological process) Relationships: is a type of GO:0042337; is part of instar larval development [GO:0002168] Also known as: larval cuticle anabolism, larval cuticle biosynthetic process, larval cuticle formation, larval cuticle synthesis Sources: GOC:bf, GOC:mtg_sensu, ISBN:0879694238 Definition: Synthesis and deposition of a chitin-based larval cuticle. The insect larval cuticle is a secretion from epidermal cells that is shed at each molt. An example of this is found in Drosophila melanogaster.